{
  "gene_name": "Zinc finger protein 846",
  "gene_symbol": "ZNF846",
  "gene": "UniProtKB:Q147U1",
  "term_label": "nucleus",
  "term_id": "GO:0005634"
}